scutellarein 7-methyl ether 4'-O-methyltransferase activity [GO:0102624] (molecular function) Definition: Catalysis of the reaction: S-adenosyl-L-methionine + scutellarein 7-methyl ether = H+ + ladanein + S-adenosyl-L-homocysteine. Sources: RHEA:73239 Relationships: is a type of methyltransferase activity [GO:0008168]